classical Lewy body [GO:0097414] (cellular component) Relationships: is a type of Lewy body [GO:0097413] Sources: NIF_Subcellular:sao4749542545 Definition: Cytoplasmic inclusion, 5 to 15 micrometers in diameter, with a dense core surrounded by a halo of 10 to 20 nm wide radially oriented alpha-synuclein fibrils. Also known as: brainstem Lewy body